{
  "gene_name": "Apolipoprotein C-IV",
  "term_label": "very-low-density lipoprotein particle",
  "term_id": "GO:0034361",
  "gene": "UniProtKB:P55056",
  "gene_symbol": "APOC4"
}